EP1 subtype prostaglandin E2 receptor binding [GO:0031864] (molecular function) Also known as: prostanoid EP1 receptor binding, EP1 subtype prostaglandin E2 receptor ligand Definition: Binding to an EP1 subtype prostaglandin E2 receptor. Relationships: is a type of GO:0031862 Sources: GOC:mah, GOC:nln